{
  "term_label": "receptor complex",
  "gene": "UniProtKB:P23467",
  "gene_name": "Receptor-type tyrosine-protein phosphatase beta",
  "gene_symbol": "PTPRB",
  "term_id": "GO:0043235"
}